tRNA pseudouridine(32) synthase activity [GO:0160151] (molecular function) Sources: EC:5.4.99.28 Definition: Catalysis of the reaction: uridine(32) in tRNA = pseudouridine(32) in tRNA. Relationships: is a type of tRNA pseudouridine synthase activity [GO:0106029]